{
  "gene_name": "Zinc finger protein 614",
  "gene": "UniProtKB:Q8N883",
  "term_label": "nucleus",
  "gene_symbol": "ZNF614",
  "term_id": "GO:0005634"
}